{
  "gene_name": "Coiled-coil domain-containing protein 66",
  "gene": "UniProtKB:A2RUB6",
  "term_id": "GO:0005874",
  "gene_symbol": "CCDC66",
  "term_label": "microtubule"
}